{
  "gene_name": "ATPase SWSAP1",
  "term_label": "Shu complex",
  "gene_symbol": "SWSAP1",
  "term_id": "GO:0097196",
  "gene": "UniProtKB:Q6NVH7"
}